D-arabinose 1-dehydrogenase (NADP+) activity [GO:0106271] (molecular function) Definition: Catalysis of the reaction: D-arabinose + NADP+ = D-arabinono-1,4-lactone + NADPH. Sources: RHEA:21892 Relationships: is a type of D-arabinose 1-dehydrogenase [NAD(P)+] activity [GO:0045290]